neurotransmitter reuptake [GO:0098810] (biological process) Sources: GOC:dos Relationships: is_a neurotransmitter uptake [GO:0001504]; is a type of establishment of localization in cell [GO:0051649]; occurs in presynapse [GO:0098793] Definition: The directed movement of neurotransmitter molecules from the extrasynaptic space into the presynaptic cytosol. Subtypes: serotonin uptake [GO:0051610], GO:0051933, catecholamine uptake involved in synaptic transmission [GO:0051934]